{
  "term_id": "GO:0000070",
  "gene": "UniProtKB:Q9Y448",
  "term_label": "mitotic sister chromatid segregation",
  "gene_name": "Small kinetochore-associated protein",
  "gene_symbol": "KNSTRN"
}